{
  "gene": "UniProtKB:Q496A3",
  "gene_name": "Spermatogenesis-associated serine-rich protein 1",
  "term_label": "Unknown biological process",
  "gene_symbol": "SPATS1",
  "term_id": "UNKNOWN:0002"
}